{
  "gene_symbol": "BCL2L11",
  "term_id": "GO:0043065",
  "gene_name": "Bcl-2-like protein 11",
  "gene": "UniProtKB:O43521",
  "term_label": "positive regulation of apoptotic process"
}